{
  "term_label": "Unknown biological process",
  "gene_symbol": "CDKN2AIPNL",
  "gene": "UniProtKB:Q96HQ2",
  "gene_name": "CDKN2AIP N-terminal-like protein",
  "term_id": "UNKNOWN:0002"
}